{
  "term_label": "Unknown biological process",
  "gene_symbol": "PKD1L1-AS1",
  "gene": "UniProtKB:Q9H7B7",
  "term_id": "UNKNOWN:0002",
  "gene_name": "Putative uncharacterized protein PKD1L1-AS1"
}